{
  "term_label": "PRC1 complex",
  "gene_symbol": "CBX4",
  "gene_name": "E3 SUMO-protein ligase CBX4",
  "term_id": "GO:0035102",
  "gene": "UniProtKB:O00257"
}